{
  "term_id": "GO:0032813",
  "gene_symbol": "TNFSF9",
  "gene": "UniProtKB:P41273",
  "gene_name": "Tumor necrosis factor ligand superfamily member 9",
  "term_label": "tumor necrosis factor receptor superfamily binding"
}